{
  "term_label": "anaphase-promoting complex binding",
  "gene_name": "Cell division cycle protein 20 homolog",
  "term_id": "GO:0010997",
  "gene": "UniProtKB:Q12834",
  "gene_symbol": "CDC20"
}